{
  "gene": "UniProtKB:Q5TEC6",
  "term_label": "nucleus",
  "term_id": "GO:0005634",
  "gene_name": "Histone H3-7",
  "gene_symbol": "H3-7"
}